{
  "term_id": "GO:0042026",
  "gene_name": "Alpha-crystallin B chain",
  "gene_symbol": "CRYAB",
  "gene": "UniProtKB:P02511",
  "term_label": "protein refolding"
}